{
  "gene": "UniProtKB:Q8IZA0",
  "gene_symbol": "KIAA0319L",
  "gene_name": "Dyslexia-associated protein KIAA0319-like protein",
  "term_id": "GO:0016020",
  "term_label": "membrane"
}